{
  "gene": "UniProtKB:Q16795",
  "term_label": "mitochondrion",
  "term_id": "GO:0005739",
  "gene_name": "NADH dehydrogenase [ubiquinone] 1 alpha subcomplex subunit 9, mitochondrial",
  "gene_symbol": "NDUFA9"
}